protein insertion into mitochondrial inner membrane [GO:0045039] (biological process) Also known as: mitochondrial inner membrane protein import, protein import into mitochondrial inner membrane, protein transport into mitochondrial inner membrane References: PMID:18672008 Sources: GOC:mcc, GOC:vw Definition: The processes mediating the insertion of proteins into the mitochondrial inner membrane. Mitochondrial inner membrane proteins can get inserted from the cytosol, by crossing the outer membrane and being guided by an inner membrane translocase complex into their final destination in the inner membrane. Some proteins present in the intermembrane space can get inserted into the inner mitochondrial membrane. Finally, some proteins are inserted into the inner membrane from the matrix side of the membrane. Subtypes: protein insertion into mitochondrial inner membrane from matrix [GO:0032979] Relationships: is a type of inner mitochondrial membrane organization [GO:0007007]; is a type of protein insertion into mitochondrial membrane [GO:0051204]